{
  "term_id": "UNKNOWN:0001",
  "term_label": "Unknown molecular function",
  "gene_symbol": "SDCCAG8",
  "gene": "UniProtKB:Q86SQ7",
  "gene_name": "Serologically defined colon cancer antigen 8"
}